dicarboxylic acid transmembrane transporter activity [GO:0005310] (molecular function) Subtypes: bilirubin transmembrane transporter activity [GO:0015127], oxaloacetate transmembrane transporter activity [GO:0015131], fumarate transmembrane transporter activity [GO:0015138], alpha-ketoglutarate transmembrane transporter activity [GO:0015139], GO:0015140, succinate transmembrane transporter activity [GO:0015141], L-aspartate transmembrane transporter activity [GO:0015183], methotrexate transmembrane transporter activity [GO:0015350], dicarboxylate:phosphate antiporter activity [GO:0015364], secondary active p-aminobenzoyl-glutamate transmembrane transporter activity [GO:0015558], sodium:dicarboxylate symporter activity [GO:0017153], oxalate transmembrane transporter activity [GO:0019531], GO:0034658, D-glucarate transmembrane transporter activity [GO:0042878], aspartate:alanine antiporter activity [GO:0070906], D-aspartate transmembrane transporter activity [GO:0140010], malonate(1-) transmembrane transporter activity [GO:1901239] Also known as: dicarboxylate carrier, sodium:dicarboxylate/tricarboxylate symporter activity, dicarboxylate (succinate/fumarate/malate) antiporter activity, dicarboxylic acid permease activity Sources: GOC:ai Relationships: is a type of carboxylic acid transmembrane transporter activity [GO:0046943]; is part of GO:0006835 Definition: Enables the transfer of dicarboxylic acids from one side of a membrane to the other. A dicarboxylic acid is an organic acid with two COOH groups.